{
  "gene_symbol": "EXOC1",
  "gene": "UniProtKB:Q9NV70",
  "term_id": "GO:0006887",
  "term_label": "exocytosis",
  "gene_name": "Exocyst complex component 1"
}